ripoptosome assembly [GO:0097343] (biological process) References: PMID:22274400 Sources: GOC:mtg_apoptosis Subtypes: ripoptosome assembly involved in extrinsic apoptotic signaling pathway [GO:1901025], ripoptosome assembly involved in necroptotic process [GO:1901026] Relationships: is a type of protein-containing complex assembly [GO:0065003] Definition: The aggregation, arrangement and bonding together of a set of components to form a ripoptosome, a protein complex whose formation can induce an extrinsic apoptotic signaling pathway or a necroptotic signaling pathway. The composition of this protein complex may depend on several factors including nature of the signal, cell type and more.